leukotriene A4 catabolic process [GO:1901752] (biological process) Definition: The chemical reactions and pathways resulting in the breakdown of leukotriene A4. Relationships: is a type of leukotriene catabolic process [GO:0036100]; is a type of GO:0042758; is a type of ether catabolic process [GO:1901502]; is a type of icosanoid catabolic process [GO:1901523]; is_a leukotriene A4 metabolic process [GO:1901751] Sources: GOC:TermGenie, GOC:yaf Also known as: leukotriene A4 breakdown, leukotriene A4 catabolism, leukotriene A4 degradation